{
  "term_label": "microtubule binding",
  "gene_name": "Regulator of microtubule dynamics protein 3",
  "gene_symbol": "RMDN3",
  "term_id": "GO:0008017",
  "gene": "UniProtKB:Q96TC7"
}